{
  "term_id": "UNKNOWN:0001",
  "gene": "UniProtKB:Q14764",
  "gene_name": "Major vault protein",
  "gene_symbol": "MVP",
  "term_label": "Unknown molecular function"
}